{
  "gene_name": "Leukemia inhibitory factor",
  "term_id": "GO:0045595",
  "gene_symbol": "LIF",
  "term_label": "regulation of cell differentiation",
  "gene": "UniProtKB:P15018"
}